{
  "gene": "UniProtKB:Q8N1Q1",
  "term_id": "UNKNOWN:0002",
  "gene_symbol": "CA13",
  "gene_name": "Carbonic anhydrase 13",
  "term_label": "Unknown biological process"
}